{
  "gene": "UniProtKB:O75896",
  "term_id": "GO:0006954",
  "term_label": "inflammatory response",
  "gene_name": "Tumor suppressor candidate 2",
  "gene_symbol": "TUSC2"
}